{
  "gene": "UniProtKB:Q99958",
  "gene_name": "Forkhead box protein C2",
  "gene_symbol": "FOXC2",
  "term_id": "GO:0006357",
  "term_label": "regulation of transcription by RNA polymerase II"
}